symbiont-mediated perturbation of host intracellular transport [GO:0052038] (biological process) Also known as: modulation by symbiont of host intracellular transport, modulation of host intracellular trafficking Subtypes: GO:0039522 Relationships: is_a symbiont-mediated perturbation of host cellular process [GO:0044068] Definition: A process in which a symbiont alters or subverts the directed movement of substances within the cell of the host organism. The host is defined as the larger of the organisms involved in a symbiotic interaction. Sources: GOC:mtg_pamgo_17jul06